thymocyte apoptotic process [GO:0070242] (biological process) Regulation: regulated by regulation of thymocyte apoptotic process [GO:0070243]; negatively regulated by negative regulation of thymocyte apoptotic process [GO:0070244]; positively regulated by GO:0070245 Note: Note that a thymocyte is an immature T cell located in the thymus (CL:0000893). Also known as: thymocyte apoptosis, immature T cell apoptosis Definition: Any apoptotic process in a thymocyte, an immature T cell located in the thymus. Sources: CL:0000893, GOC:add, GOC:mtg_apoptosis, ISBN:0781765196 Relationships: is a type of GO:0070231